{
  "term_id": "GO:0005764",
  "gene": "UniProtKB:Q0VGL1",
  "gene_name": "Ragulator complex protein LAMTOR4",
  "term_label": "lysosome",
  "gene_symbol": "LAMTOR4"
}